{
  "term_label": "centrosome",
  "gene": "UniProtKB:Q9NRH3",
  "gene_name": "Tubulin gamma-2 chain",
  "gene_symbol": "TUBG2",
  "term_id": "GO:0005813"
}